{
  "gene_name": "5-hydroxytryptamine receptor 3D",
  "term_id": "GO:0042391",
  "term_label": "regulation of membrane potential",
  "gene_symbol": "HTR3D",
  "gene": "UniProtKB:Q70Z44"
}